purine nucleobase salvage [GO:0043096] (biological process) Definition: Any process that generates purine nucleobases, one of the two classes of nitrogen-containing ring compounds found in DNA and RNA, from derivatives of them without de novo synthesis. Subtypes: adenine salvage [GO:0006168], guanine salvage [GO:0006178], hypoxanthine salvage [GO:0043103] Sources: GOC:jl Also known as: purine base salvage Relationships: is_a purine nucleobase biosynthetic process [GO:0009113]; is a type of purine-containing compound salvage [GO:0043101]